{
  "gene_symbol": "SMCR8",
  "gene_name": "Guanine nucleotide exchange protein SMCR8",
  "term_label": "Unknown biological process",
  "gene": "UniProtKB:Q8TEV9",
  "term_id": "UNKNOWN:0002"
}